{
  "term_label": "Unknown biological process",
  "gene_name": "Protein FAM167B",
  "gene": "UniProtKB:Q9BTA0",
  "gene_symbol": "FAM167B",
  "term_id": "UNKNOWN:0002"
}